secretory granule lumen [GO:0034774] (cellular component) Subtypes: GO:0031089, GO:0031093, chromaffin granule lumen [GO:0034466], GO:0035578, GO:0035580, acrosomal lumen [GO:0043160], GO:0098898 Sources: GOC:rph Relationships: is a type of GO:0060205; is part of secretory granule [GO:0030141] Definition: The volume enclosed by the membrane of a secretory granule.